{
  "term_label": "Unknown cellular component",
  "term_id": "UNKNOWN:0003",
  "gene_symbol": "TP53AIP1",
  "gene": "UniProtKB:Q9HCN2",
  "gene_name": "p53-regulated apoptosis-inducing protein 1"
}